{
  "term_label": "cilium assembly",
  "gene_name": "Tektin-1",
  "term_id": "GO:0060271",
  "gene": "UniProtKB:Q969V4",
  "gene_symbol": "TEKT1"
}